{
  "gene_symbol": "DHPS",
  "term_id": "GO:0008216",
  "term_label": "spermidine metabolic process",
  "gene_name": "Deoxyhypusine synthase",
  "gene": "UniProtKB:P49366"
}